{
  "term_id": "UNKNOWN:0003",
  "term_label": "Unknown cellular component",
  "gene_symbol": "ZBTB4",
  "gene": "UniProtKB:Q9P1Z0",
  "gene_name": "Zinc finger and BTB domain-containing protein 4"
}